{
  "gene": "UniProtKB:Q8NAA4",
  "term_id": "UNKNOWN:0001",
  "gene_symbol": "ATG16L2",
  "gene_name": "Protein Atg16l2",
  "term_label": "Unknown molecular function"
}